{
  "gene_symbol": "RHEBL1",
  "term_label": "positive regulation of TORC1 signaling",
  "term_id": "GO:1904263",
  "gene": "UniProtKB:Q8TAI7",
  "gene_name": "GTPase RhebL1"
}